{
  "term_id": "UNKNOWN:0001",
  "gene_symbol": "GTF3C1",
  "term_label": "Unknown molecular function",
  "gene_name": "General transcription factor 3C polypeptide 1",
  "gene": "UniProtKB:Q12789"
}